{
  "gene": "UniProtKB:Q8WXS5",
  "gene_name": "Voltage-dependent calcium channel gamma-8 subunit",
  "term_id": "GO:0051968",
  "gene_symbol": "CACNG8",
  "term_label": "positive regulation of synaptic transmission, glutamatergic"
}